{
  "gene_name": "EMILIN-1",
  "term_label": "Unknown cellular component",
  "gene_symbol": "EMILIN1",
  "term_id": "UNKNOWN:0003",
  "gene": "UniProtKB:Q9Y6C2"
}